{
  "term_id": "GO:0004984",
  "gene_symbol": "OR14L1",
  "gene_name": "Olfactory receptor 14L1",
  "gene": "UniProtKB:Q8NHC6",
  "term_label": "olfactory receptor activity"
}